{
  "gene_name": "Tumor necrosis factor receptor superfamily member 19",
  "term_label": "positive regulation of canonical NF-kappaB signal transduction",
  "term_id": "GO:0043123",
  "gene_symbol": "TNFRSF19",
  "gene": "UniProtKB:Q9NS68"
}